{
  "term_id": "GO:0035925",
  "gene_name": "Exosome complex component RRP45",
  "gene_symbol": "EXOSC9",
  "term_label": "mRNA 3'-UTR AU-rich region binding",
  "gene": "UniProtKB:Q06265"
}